pirellulosome [GO:0044223] (cellular component) References: PMID:19133117 Sources: GOC:dh Definition: A cytoplasmic structure found in bacterial phyla Planctomycetes and Verrucomicrobia containing a condensed nucleoid and ribosomes and surrounded by an intracytoplasmic membrane. It is surrounded by ribosome-free cytoplasm, in a compartment called the paryphoplasm. Relationships: is a type of intracellular membrane-bounded organelle [GO:0043231]; is part of cytoplasm [GO:0005737]